phosphorylase kinase activity [GO:0004689] (MF) Regulation: regulated by GO:0008607 Definition: Catalysis of the reaction: 4 ATP + 2 phosphorylase b = 4 ADP + phosphorylase a. Sources: EC:2.7.11.19 Relationships: is a type of calcium/calmodulin-dependent protein kinase activity [GO:0004683] Also known as: phosphorylase kinase, intrinsic catalyst activity, ATP:phosphorylase-b phosphotransferase activity, PHK, STK17, dephosphophosphorylase kinase activity, glycogen phosphorylase kinase activity, phosphorylase B kinase activity, phosphorylase kinase (phosphorylating) activity